{
  "term_label": "plasma membrane",
  "gene_name": "Phospholipid phosphatase 1",
  "gene": "UniProtKB:O14494",
  "gene_symbol": "PLPP1",
  "term_id": "GO:0005886"
}